{
  "gene_symbol": "C4orf36",
  "term_id": "UNKNOWN:0001",
  "term_label": "Unknown molecular function",
  "gene": "UniProtKB:Q96KX1",
  "gene_name": "Uncharacterized protein C4orf36"
}